{
  "gene_name": "Electron transfer flavoprotein beta subunit lysine methyltransferase",
  "gene": "UniProtKB:Q8IXQ9",
  "gene_symbol": "ETFBKMT",
  "term_label": "mitochondrial matrix",
  "term_id": "GO:0005759"
}